{
  "term_id": "GO:0043025",
  "gene": "UniProtKB:P41217",
  "gene_name": "OX-2 membrane glycoprotein",
  "term_label": "neuronal cell body",
  "gene_symbol": "CD200"
}